{
  "gene_name": "Ras-related GTP-binding protein A",
  "term_label": "GTP binding",
  "gene_symbol": "RRAGA",
  "term_id": "GO:0005525",
  "gene": "UniProtKB:Q7L523"
}